positive regulation of lens fiber cell differentiation [GO:1902748] (biological process) Definition: Any process that activates or increases the frequency, rate or extent of lens fiber cell differentiation. Relationships: is a type of GO:0030858; is a type of positive regulation of multicellular organismal process [GO:0051240]; is a type of GO:1902746; positively regulates lens fiber cell differentiation [GO:0070306] Also known as: positive regulation of lens fibre cell differentiation, up regulation of lens fiber cell differentiation, up regulation of lens fibre cell differentiation, up-regulation of lens fiber cell differentiation, up-regulation of lens fibre cell differentiation, upregulation of lens fiber cell differentiation, upregulation of lens fibre cell differentiation, activation of lens fiber cell differentiation, activation of lens fibre cell differentiation References: PMID:17592637 Sources: GOC:TermGenie, GOC:mr, GO_REF:0000058